{
  "gene_name": "Leptin",
  "term_label": "leptin receptor binding",
  "gene": "UniProtKB:P41159",
  "gene_symbol": "LEP",
  "term_id": "GO:1990460"
}